{
  "gene_symbol": "SYT15",
  "term_id": "GO:0005886",
  "gene_name": "Synaptotagmin-15",
  "gene": "UniProtKB:Q9BQS2",
  "term_label": "plasma membrane"
}